{
  "gene": "UniProtKB:O95050",
  "term_id": "UNKNOWN:0002",
  "gene_symbol": "INMT",
  "term_label": "Unknown biological process",
  "gene_name": "Indolethylamine N-methyltransferase"
}